{
  "term_id": "GO:0007608",
  "gene_name": "Olfactory receptor 8B3",
  "term_label": "sensory perception of smell",
  "gene": "UniProtKB:Q8NGG8",
  "gene_symbol": "OR8B3"
}